regulation of cell junction assembly [GO:1901888] (biological process) Subtypes: regulation of synapse assembly [GO:0051963], regulation of cell-substrate junction assembly [GO:0090109], GO:1901889, positive regulation of cell junction assembly [GO:1901890], regulation of gap junction assembly [GO:1903596], regulation of bicellular tight junction assembly [GO:2000810] Definition: Any process that modulates the frequency, rate or extent of cell junction assembly. Relationships: is a type of regulation of cellular component biogenesis [GO:0044087]; is a type of regulation of cellular component organization [GO:0051128]; regulates cell junction assembly [GO:0034329] Sources: GOC:TermGenie